mammary gland cord morphogenesis [GO:0060652] (biological process) Definition: The process in which anatomical structures of the mammary gland cord are generated and organized. Mammary gland cords form when the mammary gland bud invades the mammary fat. Relationships: is a type of epithelial tube morphogenesis [GO:0060562]; is part of mammary gland duct morphogenesis [GO:0060603] Also known as: mammary gland sprout morphogenesis References: PMID:12558599 Sources: GOC:dph